{
  "term_id": "GO:0019770",
  "term_label": "IgG receptor activity",
  "gene_symbol": "FCGR2C",
  "gene_name": "Low affinity immunoglobulin gamma Fc region receptor II-c",
  "gene": "UniProtKB:P31995"
}